{
  "term_id": "GO:0030335",
  "gene_name": "C-C motif chemokine 26",
  "gene_symbol": "CCL26",
  "term_label": "positive regulation of cell migration",
  "gene": "UniProtKB:Q9Y258"
}